{
  "term_label": "synaptic vesicle",
  "term_id": "GO:0008021",
  "gene": "UniProtKB:P0C0E4",
  "gene_symbol": "RAB40AL",
  "gene_name": "Ras-related protein Rab-40A-like"
}